{
  "gene_name": "TBC1 domain family member 21",
  "term_id": "GO:0005096",
  "gene": "UniProtKB:Q8IYX1",
  "gene_symbol": "TBC1D21",
  "term_label": "GTPase activator activity"
}